{
  "gene_name": "Glutamate receptor ionotropic, kainate 5",
  "term_id": "GO:0050804",
  "gene_symbol": "GRIK5",
  "term_label": "modulation of chemical synaptic transmission",
  "gene": "UniProtKB:Q16478"
}